thiamine-containing compound catabolic process [GO:0042725] (biological process) Also known as: thiamin and derivative catabolic process, thiamin and derivative catabolism, thiamin-containing compound catabolic process, thiamine and derivative catabolic process, thiamine and derivative catabolism, thiamine-containing compound breakdown, thiamine-containing compound catabolism, thiamine-containing compound degradation, vitamin B1 and derivative catabolic process, vitamin B1 and derivative catabolism Sources: GOC:jl Subtypes: GO:0009230, thiamine diphosphate catabolic process [GO:0042358] Definition: The chemical reactions and pathways resulting in the breakdown of thiamine (vitamin B1), and compounds derived from it. Relationships: is a type of water-soluble vitamin catabolic process [GO:0042365]; is a type of thiamine-containing compound metabolic process [GO:0042723]; is a type of GO:0044273; is a type of pyrimidine-containing compound catabolic process [GO:0072529]